regulation of mitotic DNA damage checkpoint [GO:1904289] (biological process) Subtypes: negative regulation of mitotic DNA damage checkpoint [GO:1904290], positive regulation of mitotic DNA damage checkpoint [GO:1904291] Relationships: is a type of regulation of mitotic cell cycle [GO:0007346]; is a type of GO:2000001; regulates mitotic DNA damage checkpoint signaling [GO:0044773] Definition: Any process that modulates the frequency, rate or extent of mitotic DNA damage checkpoint. References: PMID:16549501 Sources: GOC:TermGenie, GOC:kmv, GO_REF:0000058